{
  "gene": "UniProtKB:Q8N8B7",
  "gene_name": "Transcription elongation factor A N-terminal and central domain-containing protein",
  "term_label": "transcription elongation by RNA polymerase II",
  "gene_symbol": "TCEANC",
  "term_id": "GO:0006368"
}